{
  "gene_name": "Malignant T-cell-amplified sequence 2",
  "gene_symbol": "MCTS2",
  "term_id": "UNKNOWN:0003",
  "term_label": "Unknown cellular component",
  "gene": "UniProtKB:A0A3B3IRV3"
}